{
  "term_id": "UNKNOWN:0002",
  "gene": "UniProtKB:Q8NAQ8",
  "gene_name": "Putative uncharacterized protein FLJ34945",
  "term_label": "Unknown biological process",
  "gene_symbol": "Q8NAQ8"
}